{
  "gene": "UniProtKB:Q8N5K1",
  "term_id": "GO:0000422",
  "term_label": "autophagy of mitochondrion",
  "gene_symbol": "CISD2",
  "gene_name": "CDGSH iron-sulfur domain-containing protein 2"
}